{
  "term_id": "GO:0005743",
  "gene_symbol": "OXA1L",
  "gene_name": "Mitochondrial inner membrane protein OXA1L",
  "gene": "UniProtKB:Q15070",
  "term_label": "mitochondrial inner membrane"
}